{
  "term_label": "nucleus",
  "term_id": "GO:0005634",
  "gene_name": "Anomalous homeobox protein",
  "gene": "UniProtKB:E9PGG2",
  "gene_symbol": "ANHX"
}